{
  "term_label": "Unknown molecular function",
  "gene_symbol": "VCX",
  "term_id": "UNKNOWN:0001",
  "gene": "UniProtKB:Q9H320",
  "gene_name": "Variable charge X-linked protein 1"
}